{
  "term_id": "GO:0014069",
  "gene": "UniProtKB:Q9NQC3",
  "term_label": "postsynaptic density",
  "gene_symbol": "RTN4",
  "gene_name": "Reticulon-4"
}